{
  "term_label": "cytoplasm",
  "gene_symbol": "MX2",
  "term_id": "GO:0005737",
  "gene": "UniProtKB:P20592",
  "gene_name": "Interferon-induced GTP-binding protein Mx2"
}